{
  "term_id": "GO:0007507",
  "gene": "UniProtKB:P36382",
  "gene_symbol": "GJA5",
  "gene_name": "Gap junction alpha-5 protein",
  "term_label": "heart development"
}